dense core granule [GO:0031045] (cellular component) Subtypes: neuronal dense core vesicle [GO:0098992] References: PMID:14690495 Sources: NIF_Subcellular:sao772007592 Relationships: is a type of GO:0030141 Definition: Electron-dense organelle with a granular internal matrix; contains proteins destined to be secreted. Also known as: dense core vesicle